{
  "gene_symbol": "KATNA1",
  "gene_name": "Katanin p60 ATPase-containing subunit A1",
  "term_label": "microtubule severing ATPase activity",
  "gene": "UniProtKB:O75449",
  "term_id": "GO:0008568"
}